{
  "term_label": "nucleus",
  "gene_symbol": "SS18",
  "term_id": "GO:0005634",
  "gene_name": "Protein SSXT",
  "gene": "UniProtKB:Q15532"
}